lymphocyte adhesion to endothelial cell of high endothelial venule [GO:0036339] (biological process) Definition: The attachment of a lymphocyte to an endothelial cell of a high endothelial venule (HEV) via adhesion molecules. A HEV cell is an endothelial cell that is cuboidal, expresses leukocyte-specific receptors, and allows for passage of lymphocytes into bloodstream. Also known as: lymphocyte adhesion to HEV cell, lymphocyte adhesion to high endothelial venule Note: For the transition of leukocytes from rolling to adhered, consider instead annotating to 'leukocyte adhesive activation ; GO:0050902'. References: PMID:19339990, PMID:7679710 Sources: CL:0000542, CL:0002652, GOC:nhn, Wikipedia:High_endothelial_venules Relationships: is a type of leukocyte adhesion to vascular endothelial cell [GO:0061756]